positive regulation of mechanoreceptor differentiation [GO:0045633] (biological process) Also known as: up regulation of mechanoreceptor differentiation, up-regulation of mechanoreceptor differentiation, upregulation of mechanoreceptor differentiation, activation of mechanoreceptor differentiation, stimulation of mechanoreceptor differentiation Definition: Any process that activates or increases the frequency, rate or extent of mechanoreceptor differentiation. Relationships: is a type of regulation of mechanoreceptor differentiation [GO:0045631]; is a type of positive regulation of neuron differentiation [GO:0045666]; positively regulates mechanoreceptor differentiation [GO:0042490] Subtypes: positive regulation of inner ear receptor cell differentiation [GO:2000982] Sources: GOC:go_curators